{
  "gene_name": "Protein ABHD12B",
  "gene": "UniProtKB:Q7Z5M8",
  "term_id": "GO:0004622",
  "term_label": "phosphatidylcholine lysophospholipase activity",
  "gene_symbol": "ABHD12B"
}